response to interferon-beta [GO:0035456] (biological process) Also known as: response to fiblaferon, response to fibroblast interferon, response to interferon beta, response to beta-1 interferon References: PMID:9561374 Sources: GOC:sl Definition: Any process that results in a change in state or activity of a cell or an organism (in terms of movement, secretion, enzyme production, gene expression, etc.) as a result of an interferon-beta stimulus. Interferon-beta is a type I interferon. Subtypes: cellular response to interferon-beta [GO:0035458] Relationships: is a type of response to cytokine [GO:0034097]